negative regulation of protein geranylgeranylation [GO:2000540] (BP) Also known as: negative regulation of protein amino acid geranylgeranylation, negative regulation of C-terminal protein geranylgeranylation Definition: Any process that stops, prevents or reduces the frequency, rate or extent of protein geranylgeranylation. Sources: GOC:obol Relationships: is a type of negative regulation of protein modification process [GO:0031400]; is a type of regulation of protein geranylgeranylation [GO:2000539]; negatively regulates protein geranylgeranylation [GO:0018344]